{
  "term_label": "eosinophil chemotaxis",
  "gene": "UniProtKB:O00626",
  "term_id": "GO:0048245",
  "gene_symbol": "CCL22",
  "gene_name": "C-C motif chemokine 22"
}